positive regulation of protein modification by small protein conjugation or removal [GO:1903322] (biological process) Definition: Any process that activates or increases the frequency, rate or extent of protein modification by small protein conjugation or removal. Also known as: up regulation of protein modification by small protein conjugation or removal, up-regulation of protein modification by small protein conjugation or removal, upregulation of protein modification by small protein conjugation or removal, activation of protein modification by small protein conjugation or removal Relationships: is a type of positive regulation of post-translational protein modification [GO:1901875]; is a type of regulation of protein modification by small protein conjugation or removal [GO:1903320]; positively regulates GO:0070647 Sources: GOC:TermGenie, GOC:vw, GO_REF:0000058 Subtypes: positive regulation of protein ubiquitination [GO:0031398], positive regulation of protein sumoylation [GO:0033235], positive regulation of protein desumoylation [GO:0060189], positive regulation of protein deubiquitination [GO:1903003], GO:2000436